{
  "term_label": "GTPase activator activity",
  "gene_symbol": "ADAP2",
  "gene_name": "Arf-GAP with dual PH domain-containing protein 2",
  "gene": "UniProtKB:Q9NPF8",
  "term_id": "GO:0005096"
}